{
  "gene_symbol": "COMMD8",
  "gene": "UniProtKB:Q9NX08",
  "term_label": "Unknown cellular component",
  "gene_name": "COMM domain-containing protein 8",
  "term_id": "UNKNOWN:0003"
}